Rpd3S complex [GO:0032221] (CC) Also known as: Clr6 histone deacetylase complex II, Clr6 histone deacetylase complex II', Clr6-CII complex, Clr6S complex, Rpd3C(S), Rpd3S, Sin3S Definition: A eukaryotically conserved histone deacetylase complex which deacetylates histones across gene coding regions. Composed of a catalytic histone deacetylase subunit, a chromodomain protein, a SIN3 family co-repressor, and a WD repeat protein (Clr6p, Alp13p, Pst2p, and Prw1p respectively in Schizosaccharomyces; Rpd3p, Sin3p, Ume1p, Rco1p and Eaf3 in Saccharomyces; homologs thereof in other species). Relationships: is a type of Sin3-type complex [GO:0070822] References: PMID:12773392, PMID:17450151 Sources: GOC:vw